{
  "term_label": "Unknown molecular function",
  "gene_symbol": "PDE6H",
  "gene": "UniProtKB:Q13956",
  "term_id": "UNKNOWN:0001",
  "gene_name": "Retinal cone rhodopsin-sensitive cGMP 3',5'-cyclic phosphodiesterase subunit gamma"
}